{
  "gene_name": "Acyl-coenzyme A thioesterase 8",
  "gene_symbol": "ACOT8",
  "gene": "UniProtKB:O14734",
  "term_id": "GO:0047617",
  "term_label": "fatty acyl-CoA hydrolase activity"
}